{
  "term_label": "somitogenesis",
  "gene": "UniProtKB:Q06190",
  "gene_symbol": "PPP2R3A",
  "term_id": "GO:0001756",
  "gene_name": "Serine_threonine-protein phosphatase 2A regulatory subunit B'' subunit alpha"
}